{
  "gene_symbol": "LYZL1",
  "gene": "UniProtKB:Q6UWQ5",
  "term_label": "Unknown cellular component",
  "term_id": "UNKNOWN:0003",
  "gene_name": "Lysozyme-like protein 1"
}